{
  "gene_name": "Complex I assembly factor TIMMDC1, mitochondrial",
  "term_label": "Unknown biological process",
  "gene_symbol": "TIMMDC1",
  "gene": "UniProtKB:Q9NPL8",
  "term_id": "UNKNOWN:0002"
}